{
  "gene_symbol": "MEIOB",
  "term_label": "resolution of meiotic recombination intermediates",
  "gene": "UniProtKB:Q8N635",
  "term_id": "GO:0000712",
  "gene_name": "Meiosis-specific with OB domain-containing protein"
}